{
  "gene_symbol": "KLHL20",
  "gene_name": "Kelch-like protein 20",
  "gene": "UniProtKB:Q9Y2M5",
  "term_label": "Cul3-RING ubiquitin ligase complex",
  "term_id": "GO:0031463"
}